{
  "term_label": "cytosolic small ribosomal subunit",
  "gene": "UniProtKB:Q8TD47",
  "gene_name": "Small ribosomal subunit protein eS4, Y isoform 2",
  "gene_symbol": "RPS4Y2",
  "term_id": "GO:0022627"
}